{
  "gene_symbol": "POLR2K",
  "gene_name": "DNA-directed RNA polymerases I, II, and III subunit RPABC4",
  "gene": "UniProtKB:P53803",
  "term_id": "GO:0005666",
  "term_label": "RNA polymerase III complex"
}